{
  "gene_symbol": "HSP90AB3P",
  "term_id": "GO:0005524",
  "gene_name": "Putative heat shock protein HSP 90-beta-3",
  "term_label": "ATP binding",
  "gene": "UniProtKB:Q58FF7"
}